nucleolar peripheral inclusion body [GO:0140602] (cellular component) Also known as: NuRs, nucleolar rings Relationships: is a type of nuclear inclusion body [GO:0042405] Definition: Inclusion bodies located at the nucleolar periphery where several nuclear factors are reversibly aggregated and sequestered during acute heat stress or starvation. References: PMID:33176152, PMID:37128864